{
  "term_label": "Unknown cellular component",
  "gene": "UniProtKB:P0DTU3",
  "gene_symbol": "TRA",
  "gene_name": "T cell receptor alpha chain MC.7.G5",
  "term_id": "UNKNOWN:0003"
}